{
  "gene_symbol": "ZNRF4",
  "gene": "UniProtKB:Q8WWF5",
  "term_id": "GO:0005737",
  "gene_name": "E3 ubiquitin-protein ligase ZNRF4",
  "term_label": "cytoplasm"
}